{
  "term_id": "GO:0000977",
  "term_label": "RNA polymerase II transcription regulatory region sequence-specific DNA binding",
  "gene_name": "Homeobox protein cut-like 1",
  "gene_symbol": "CUX1",
  "gene": "UniProtKB:P39880"
}